peptidylamidoglycolate lyase activity [GO:0004598] (molecular function) Also known as: HGAD, PAL, PGL, alpha-hydroxyglycine amidating dealkylase activity, peptidyl-alpha-hydroxyglycine alpha-amidating lyase activity, peptidylamidoglycolate peptidylamide-lyase (glyoxylate-forming), peptidylamidoglycolate peptidylamide-lyase activity Sources: EC:4.3.2.5 Relationships: is a type of amidine-lyase activity [GO:0016842]; is a type of catalytic activity, acting on a protein [GO:0140096] Definition: Catalysis of the reaction: peptidylamidoglycolate = peptidyl amide + glyoxylate.